{
  "gene_name": "Histone H2A.Z",
  "gene_symbol": "H2AZ1",
  "term_id": "GO:0031507",
  "gene": "UniProtKB:P0C0S5",
  "term_label": "heterochromatin formation"
}